{
  "gene_name": "Transcriptional enhancer factor TEF-3",
  "gene_symbol": "TEAD4",
  "term_label": "hippo signaling",
  "gene": "UniProtKB:Q15561",
  "term_id": "GO:0035329"
}